VEGF-activated platelet-derived growth factor receptor signaling pathway [GO:0038086] (BP) Also known as: VEGF-activated PDGFR signalling pathway, VEGF-activated platelet-derived growth factor receptor signalling pathway, VEGF/PDGFR signaling pathway, vascular endothelial growth factor-activated platelet-derived growth factor receptor signaling pathway, VEGF-A/PDGFR signaling Subtypes: GO:0038087, VEGF-activated platelet-derived growth factor receptor-beta signaling pathway [GO:0038088], positive regulation of cell migration by VEGF-activated platelet derived growth factor receptor signaling pathway [GO:0038090], positive regulation of cell proliferation by VEGF-activated platelet derived growth factor receptor signaling pathway [GO:0038091] Definition: The series of molecular signals initiated by vascular endothelial growth factor (VEGF) binding to a platelet-derived growth factor receptor (PDGFR) on the surface of a cell, and ending with the regulation of a downstream cellular process, e.g. transcription. Relationships: is a type of GO:0038084; is a type of platelet-derived growth factor receptor signaling pathway [GO:0048008]; has part vascular endothelial growth factor receptor activity [GO:0005021] References: PMID:17470632 Sources: GOC:signaling